{
  "gene_symbol": "SOBP",
  "gene": "UniProtKB:A7XYQ1",
  "term_label": "Unknown molecular function",
  "term_id": "UNKNOWN:0001",
  "gene_name": "Sine oculis-binding protein homolog"
}